{
  "term_label": "Unknown cellular component",
  "gene_name": "Putative uncharacterized protein ASB16-AS1",
  "gene_symbol": "ASB16-AS1",
  "gene": "UniProtKB:Q495Z4",
  "term_id": "UNKNOWN:0003"
}